non-growing cell tip [GO:0035839] (cellular component) Sources: GOC:expert_jd, GOC:mah Relationships: is a type of cell tip [GO:0051286] Definition: A cell tip at which no growth takes place. For example, in fission yeast the cell end newly formed by cell division does not grow immediately upon its formation, and lacks actin cytoskeletal structures. Also known as: non-growing cell end, new cell end